{
  "term_label": "leukotriene-C4 synthase activity",
  "gene_symbol": "ALOX5AP",
  "gene_name": "Arachidonate 5-lipoxygenase-activating protein",
  "gene": "UniProtKB:P20292",
  "term_id": "GO:0004464"
}